amino acid metabolic process [GO:0006520] (biological process) Sources: ISBN:0198506732 Regulation: regulated by regulation of amino acid metabolic process [GO:0006521]; negatively regulated by negative regulation of amino acid metabolic process [GO:0045763]; positively regulated by positive regulation of amino acid metabolic process [GO:0045764] Also known as: cellular amino acid metabolic process, cellular amino acid metabolism, amino acid and derivative metabolism, cellular amino acid and derivative metabolic process Relationships: is a type of GO:0044238 Subtypes: amino acid biosynthetic process [GO:0008652], GO:0009063, aromatic amino acid metabolic process [GO:0009072], branched-chain amino acid metabolic process [GO:0009081], GO:0018366, carnosine metabolic process [GO:0035498], amino acid activation [GO:0043038], proteinogenic amino acid metabolic process [GO:0170039], non-proteinogenic amino acid metabolic process [GO:0170041], alpha-amino acid metabolic process [GO:1901605] Definition: The chemical reactions and pathways involving amino acids, carboxylic acids containing one or more amino groups.